{
  "gene": "UniProtKB:Q676U5",
  "term_id": "GO:0034274",
  "term_label": "Atg12-Atg5-Atg16 complex",
  "gene_symbol": "ATG16L1",
  "gene_name": "Autophagy-related protein 16-1"
}